U12-type spliceosomal complex [GO:0005689] (cellular component) References: PMID:11574683, PMID:11971955 Sources: GOC:krc, GOC:mah Also known as: minor (U12-type) spliceosomal complex, minor spliceosomal complex, AT-AC spliceosomal complex Subtypes: U12-type prespliceosome [GO:0071015], GO:0071016, U12-type catalytic step 1 spliceosome [GO:0071017], GO:0071018, U12-type post-mRNA release spliceosomal complex [GO:0071019], U12-type post-spliceosomal complex [GO:0071022] Relationships: is a type of spliceosomal complex [GO:0005681] Definition: Any spliceosomal complex that forms during the splicing of a messenger RNA primary transcript to excise an intron; the series of U12-type spliceosomal complexes is involved in the splicing of the majority of introns that contain atypical AT-AC terminal dinucleotides, as well as other non-canonical introns. The entire splice site signal, not just the terminal dinucleotides, is involved in determining which spliceosome utilizes the site.